pyramid development [GO:0072056] (biological process) Also known as: kidney pyramid development, pyramids development, renal medulla development, renal pyramid development Definition: The process whose specific outcome is the progression of the kidney pyramids over time, from its formation to the mature structure. Kidney pyramids are the conical masses that constitute the renal medulla in a multi-lobed mammalian kidney; they contain the loops of Henle and the medullary collecting ducts. Relationships: is a type of GO:0048856; is part of kidney development [GO:0001822] Sources: GOC:mtg_kidney_jan10 Subtypes: metanephric pyramids development [GO:0072211]